guanine nucleotide transmembrane transport [GO:1903790] (biological process) Relationships: is a type of GO:0001408; is a type of purine-containing compound transmembrane transport [GO:0072530]; is a type of nucleotide transmembrane transport [GO:1901679] References: PMID:25320081 Sources: GOC:TermGenie, GOC:dph, GOC:vw, GO_REF:0000069 Subtypes: cyclic-GMP-AMP transmembrane import across plasma membrane [GO:0140361] Definition: The process in which a guanyl nucleotide is transported across a membrane. Also known as: guanyl nucleotide transmembrane transport